{
  "term_id": "GO:0007416",
  "gene": "UniProtKB:O43157",
  "gene_name": "Plexin-B1",
  "term_label": "synapse assembly",
  "gene_symbol": "PLXNB1"
}